flavanone 3-dioxygenase activity [GO:0045486] (molecular function) Also known as: naringenin 3-dioxygenase activity, (2S)-flavanone 3-hydroxylase activity, flavanone 3-beta-hydroxylase activity, flavanone 3-hydroxylase activity, flavanone 3beta-hydroxylase activity, flavanone synthase I activity, flavanone,2-oxoglutarate:oxygen oxidoreductase (3-hydroxylating), naringenin 3-hydroxylase activity, naringenin,2-oxoglutarate:oxygen oxidoreductase (3-hydroxylating) activity Sources: RHEA:18621 Definition: Catalysis of the reaction: 2-oxoglutarate + a (2S)-flavan-4-one + O2 = a (2R,3R)-dihydroflavonol + CO2 + succinate. Relationships: is_a 2-oxoglutarate-dependent dioxygenase activity [GO:0016706]